cellular response to azide [GO:0097185] (biological process) Definition: Any process that results in a change in state or activity of a cell (in terms of movement, secretion, enzyme production, gene expression, etc.) as a result of an azide stimulus. References: PMID:16846222 Sources: GOC:yaf Relationships: is a type of response to azide [GO:0097184]; is a type of cellular response to nitrogen compound [GO:1901699]